hypoglossal nerve structural organization [GO:0021621] (biological process) Definition: The process that contributes to the act of creating the structural organization of the hypoglossal nerve. This process pertains to the physical shaping of a rudimentary structure. This motor nerve innervates all the intrinsic and all but one of the extrinsic muscles of the tongue. Sources: GOC:cls, GOC:dgh, GOC:dph, GOC:jid, GO_REF:0000021 Relationships: is a type of cranial nerve structural organization [GO:0021604]; is part of hypoglossal nerve morphogenesis [GO:0021618] Also known as: hypoglossal nerve structural organisation, CN XII structural organization